cytoplasmic side of endosome membrane [GO:0010009] (cellular component) Subtypes: GO:0098559, cytoplasmic side of late endosome membrane [GO:0098560] Definition: The side (leaflet) of the endosome membrane that faces the cytoplasm. Relationships: is a type of cytoplasmic side of membrane [GO:0098562]; is part of endosome membrane [GO:0010008] Also known as: external leaflet of endosome membrane, external side of endosome membrane Sources: GOC:lr